histone H3K56me2/H3K56me3 demethylase activity [GO:0140760] (molecular function) Also known as: histone H3-tri/dimethyl-lysine-56 demethylase activity, histone H3K56me2 demethylase activity, histone H3K56me3 demethylase activity, histone demethylase activity (H3-K56 specific) References: PMID:23451023, PMID:28743002 Definition: Catalysis of the removal of a methyl group from a tri or a dimethyl-lysine residue at position 56 of the histone H3 protein. Relationships: is a type of GO:0016706; is a type of histone H3 demethylase activity [GO:0141052] Note: Comment: Note that the residue position corresponds to the canonical human H3 histone (UniProtKB:P84243); this residue is conserved across all eukaryotes. Residue 1 is the first residue following removal of the initiating Methionine (Met). Note that each histone is encoded by multiple genes, and sequences may vary across different genes within an organism.